dentinogenesis [GO:0097187] (biological process) References: PMID:10206335, PMID:21196346 Sources: GOC:cjm, GOC:sl Also known as: dentin development, dentine development Relationships: is a type of GO:0042475; is a type of anatomical structure formation involved in morphogenesis [GO:0048646] Definition: The process whose specific outcome is the formation of dentin, the mineralized tissue that constitutes the major bulk of teeth. Dentin may be one of three types: primary dentin, secondary dentin, and tertiary dentin.